{
  "gene_name": "Forkhead box protein C2",
  "term_label": "cell differentiation",
  "gene": "UniProtKB:Q99958",
  "term_id": "GO:0030154",
  "gene_symbol": "FOXC2"
}